{
  "gene_name": "Zinc finger and BTB domain-containing protein 7B",
  "term_label": "Unknown cellular component",
  "gene_symbol": "ZBTB7B",
  "term_id": "UNKNOWN:0003",
  "gene": "UniProtKB:O15156"
}